{
  "gene": "UniProtKB:Q9BSE4",
  "term_label": "Unknown molecular function",
  "gene_name": "Homocysteine-responsive endoplasmic reticulum-resident ubiquitin-like domain member 2 protein",
  "term_id": "UNKNOWN:0001",
  "gene_symbol": "HERPUD2"
}